{
  "gene_name": "ATP-dependent DNA helicase Q4",
  "gene_symbol": "RECQL4",
  "term_id": "GO:0005694",
  "term_label": "chromosome",
  "gene": "UniProtKB:O94761"
}